{
  "gene_name": "Aurora kinase A and ninein-interacting protein",
  "gene_symbol": "AUNIP",
  "term_id": "GO:0007051",
  "term_label": "spindle organization",
  "gene": "UniProtKB:Q9H7T9"
}